{
  "term_id": "GO:0017101",
  "gene": "UniProtKB:Q13155",
  "gene_name": "Aminoacyl tRNA synthase complex-interacting multifunctional protein 2",
  "term_label": "aminoacyl-tRNA synthetase multienzyme complex",
  "gene_symbol": "AIMP2"
}